{
  "term_label": "spindle pole",
  "term_id": "GO:0000922",
  "gene_name": "Proline_serine-rich coiled-coil protein 1",
  "gene": "UniProtKB:Q6PGN9",
  "gene_symbol": "PSRC1"
}